{
  "term_id": "UNKNOWN:0001",
  "gene": "UniProtKB:Q9UJX4",
  "gene_name": "Anaphase-promoting complex subunit 5",
  "gene_symbol": "ANAPC5",
  "term_label": "Unknown molecular function"
}